{
  "gene": "UniProtKB:Q14952",
  "gene_symbol": "KIR2DS3",
  "term_label": "transmembrane signaling receptor activity",
  "gene_name": "Killer cell immunoglobulin-like receptor 2DS3",
  "term_id": "GO:0004888"
}